{
  "gene": "UniProtKB:Q8IVH8",
  "term_label": "cytoplasm",
  "gene_name": "Mitogen-activated protein kinase kinase kinase kinase 3",
  "gene_symbol": "MAP4K3",
  "term_id": "GO:0005737"
}